{
  "gene_name": "Trafficking kinesin-binding protein 1",
  "term_id": "GO:0050811",
  "gene_symbol": "TRAK1",
  "term_label": "GABA receptor binding",
  "gene": "UniProtKB:Q9UPV9"
}